{
  "gene_symbol": "C5orf58",
  "term_label": "Unknown molecular function",
  "gene_name": "Putative uncharacterized protein C5orf58",
  "term_id": "UNKNOWN:0001",
  "gene": "UniProtKB:C9J3I9"
}